protein carrier chaperone [GO:0140597] (molecular function) References: PMID:7628437 Subtypes: GO:0032977, lipoprotein carrier activity [GO:0140598], GO:0140713 Relationships: is a type of GO:0140104; has part protein binding [GO:0005515] Also known as: protein chaperone, protein carrier activity Definition: Binding to and carrying a protein between two different cellular components by moving along with the target protein.